{
  "term_label": "double-strand break repair via homologous recombination",
  "gene": "UniProtKB:Q9Y620",
  "gene_symbol": "RAD54B",
  "gene_name": "DNA repair and recombination protein RAD54B",
  "term_id": "GO:0000724"
}